{
  "gene_symbol": "ARPIN",
  "gene": "UniProtKB:Q7Z6K5",
  "term_label": "Unknown cellular component",
  "gene_name": "Arpin",
  "term_id": "UNKNOWN:0003"
}